{
  "gene_name": "Roquin-1",
  "gene": "UniProtKB:Q5TC82",
  "term_label": "ubiquitin protein ligase activity",
  "gene_symbol": "RC3H1",
  "term_id": "GO:0061630"
}